positive regulation of phospholipid biosynthetic process [GO:0071073] (biological process) Subtypes: positive regulation of phosphatidylinositol biosynthetic process [GO:0010513], positive regulation of phosphatidylserine biosynthetic process [GO:1900470], GO:1900486, positive regulation of phosphatidylglycerol biosynthetic process [GO:1901353], GO:1905695, positive regulation of phosphatidylcholine biosynthetic process [GO:2001247] Sources: GOC:mah Relationships: is a type of positive regulation of lipid biosynthetic process [GO:0046889]; is a type of GO:0071071; is_a positive regulation of phospholipid metabolic process [GO:1903727]; positively regulates GO:0008654 Definition: Any process that activates or increases the frequency, rate or extent of the chemical reactions and pathways resulting in the formation of phospholipids. Also known as: positive regulation of phospholipid anabolism, positive regulation of phospholipid biosynthesis, positive regulation of phospholipid formation, positive regulation of phospholipid synthesis, up regulation of phospholipid biosynthetic process, up-regulation of phospholipid biosynthetic process, upregulation of phospholipid biosynthetic process, activation of phospholipid biosynthetic process, stimulation of phospholipid biosynthetic process